{
  "gene": "UniProtKB:Q96PG1",
  "gene_symbol": "MS4A4E",
  "gene_name": "Putative membrane-spanning 4-domains subfamily A member 4E",
  "term_label": "Unknown molecular function",
  "term_id": "UNKNOWN:0001"
}